{
  "term_label": "5'-nucleotidase activity",
  "gene_symbol": "NT5C1A",
  "gene": "UniProtKB:Q9BXI3",
  "term_id": "GO:0008253",
  "gene_name": "Cytosolic 5'-nucleotidase 1A"
}